{
  "gene_symbol": "HLA-DPA1",
  "term_id": "GO:0050870",
  "gene_name": "HLA class II histocompatibility antigen, DP alpha 1 chain",
  "term_label": "positive regulation of T cell activation",
  "gene": "UniProtKB:P20036"
}